arterial endothelial cell fate commitment [GO:0060844] (biological process) Definition: The commitment of a cell to an arterial endothelial cell fate and its capacity to differentiate into an arterial endothelial cell. Relationships: is a type of blood vessel endothelial cell fate commitment [GO:0060846]; is part of arterial endothelial cell differentiation [GO:0060842] Sources: GOC:dph, GOC:sdb_2009, GOC:tb